{
  "gene": "UniProtKB:P40938",
  "term_id": "GO:0006281",
  "gene_symbol": "RFC3",
  "gene_name": "Replication factor C subunit 3",
  "term_label": "DNA repair"
}